{
  "gene_symbol": "BANF1",
  "term_label": "condensed chromosome",
  "gene_name": "Barrier-to-autointegration factor",
  "gene": "UniProtKB:O75531",
  "term_id": "GO:0000793"
}